{
  "gene": "UniProtKB:P37173",
  "gene_symbol": "TGFBR2",
  "term_label": "nervous system development",
  "gene_name": "TGF-beta receptor type-2",
  "term_id": "GO:0007399"
}